{
  "gene": "UniProtKB:Q5JTN6",
  "term_label": "Unknown molecular function",
  "gene_symbol": "WDR38",
  "term_id": "UNKNOWN:0001",
  "gene_name": "WD repeat-containing protein 38"
}